{
  "term_label": "nucleus",
  "term_id": "GO:0005634",
  "gene_name": "Cyclic AMP-dependent transcription factor ATF-3",
  "gene": "UniProtKB:P18847",
  "gene_symbol": "ATF3"
}